{
  "gene_symbol": "NTN4",
  "gene_name": "Netrin-4",
  "term_label": "cell migration",
  "term_id": "GO:0016477",
  "gene": "UniProtKB:Q9HB63"
}